definition [IAO:0000115]